{
  "gene_symbol": "ABI3BP",
  "term_id": "UNKNOWN:0003",
  "gene": "UniProtKB:Q7Z7G0",
  "term_label": "Unknown cellular component",
  "gene_name": "Target of Nesh-SH3"
}